farnesylated protein binding [GO:0001918] (molecular function) References: PMID:14555765 Sources: GOC:add Relationships: is_a protein binding [GO:0005515] Definition: Binding to a farnesylated protein.